{
  "gene_name": "Neuron navigator 1",
  "gene": "UniProtKB:Q8NEY1",
  "gene_symbol": "NAV1",
  "term_id": "GO:0015630",
  "term_label": "microtubule cytoskeleton"
}